UTP:xylose-1-phosphate uridylyltransferase activity [GO:0047338] (molecular function) Also known as: UDP-xylose pyrophosphorylase activity, UTP-xylose-1-phosphate uridylyltransferase activity, UTP:alpha-D-xylose-1-phosphate uridylyltransferase activity, uridine diphosphoxylose pyrophosphorylase activity, uridylyltransferase, xylose 1-phosphate, xylose 1-phosphate uridylyltransferase activity, xylose-1-phosphate uridylyltransferase activity Sources: EC:2.7.7.11, MetaCyc:2.7.7.11-RXN Relationships: is a type of UTP-monosaccharide-1-phosphate uridylyltransferase activity [GO:0051748] Definition: Catalysis of the reaction: alpha-D-xylose 1-phosphate + UTP = UDP-D-xylose + diphosphate.